{
  "term_id": "GO:0005737",
  "gene_name": "Numb-like protein",
  "term_label": "cytoplasm",
  "gene": "UniProtKB:Q9Y6R0",
  "gene_symbol": "NUMBL"
}